{
  "gene_symbol": "MFSD2A",
  "gene": "UniProtKB:Q8NA29",
  "term_label": "lysophospholipid:sodium symporter activity",
  "gene_name": "Sodium-dependent lysophosphatidylcholine symporter 1",
  "term_id": "GO:0051978"
}